{
  "gene_symbol": "ASB2",
  "gene": "UniProtKB:Q96Q27",
  "gene_name": "Ankyrin repeat and SOCS box protein 2",
  "term_id": "GO:0005634",
  "term_label": "nucleus"
}